cholesterol binding [GO:0015485] (molecular function) Definition: Binding to cholesterol (cholest-5-en-3-beta-ol); the principal sterol of vertebrates and the precursor of many steroids, including bile acids and steroid hormones. Relationships: is a type of sterol binding [GO:0032934]; is a type of alcohol binding [GO:0043178] Sources: GOC:jl, ISBN:0198506732